organellar chromatophore thylakoid [GO:0070116] (cellular component) Definition: A thylakoid located in an organellar chromatophore. Sources: GOC:mah Also known as: Paulinella-type chromatophore thylakoid Relationships: is a type of thylakoid [GO:0009579]; BFO_0000050 organellar chromatophore [GO:0070111]